{
  "gene": "UniProtKB:P35226",
  "gene_name": "Polycomb complex protein BMI-1",
  "term_label": "negative regulation of transcription by RNA polymerase II",
  "gene_symbol": "BMI1",
  "term_id": "GO:0000122"
}